{
  "term_label": "RNA polymerase II cis-regulatory region sequence-specific DNA binding",
  "term_id": "GO:0000978",
  "gene_symbol": "JUN",
  "gene": "UniProtKB:P05412",
  "gene_name": "Transcription factor Jun"
}